{
  "gene": "UniProtKB:P08727",
  "term_label": "intermediate filament organization",
  "gene_name": "Keratin, type I cytoskeletal 19",
  "gene_symbol": "KRT19",
  "term_id": "GO:0045109"
}